glossopharyngeal nerve formation [GO:0021616] (biological process) Relationships: is a type of cranial nerve formation [GO:0021603]; is part of glossopharyngeal nerve morphogenesis [GO:0021615] Also known as: CN IX biosynthesis, CN IX formation Definition: The process that gives rise to the glossopharyngeal nerve. This process pertains to the initial formation of a structure from unspecified parts. Various sensory and motor branches of the glossopharyngeal nerve supply nerve connections to the pharynx and back of the tongue. The branchial motor component contains motor fibers that innervate muscles that elevate the pharynx and larynx, and the tympanic branch supplies parasympathetic fibers to the otic ganglion. Sources: GOC:cls, GOC:dgh, GOC:dph, GOC:jid, GO_REF:0000021